{
  "gene_name": "Phosphatidylinositol 4-phosphate 3-kinase C2 domain-containing subunit beta",
  "term_label": "phosphatidylinositol-mediated signaling",
  "term_id": "GO:0048015",
  "gene_symbol": "PIK3C2B",
  "gene": "UniProtKB:O00750"
}